flight involved in flight behavior [GO:0060362] (biological process) Definition: Self-propelled movement of an organism from one location to another through the air that is part of the organism's response to external or internal stimuli resulting in flight. Relationships: is a type of locomotion involved in locomotory behavior [GO:0031987]; is a type of GO:0060361; is part of GO:0007629 Sources: GOC:dph